{
  "term_label": "ceramide biosynthetic process",
  "gene_symbol": "AGK",
  "gene": "UniProtKB:Q53H12",
  "gene_name": "Acylglycerol kinase, mitochondrial",
  "term_id": "GO:0046513"
}